{
  "term_label": "Unknown molecular function",
  "gene": "UniProtKB:Q1L6U9",
  "gene_name": "Prostate-associated microseminoprotein",
  "term_id": "UNKNOWN:0001",
  "gene_symbol": "MSMP"
}